positive regulation of RNA splicing [GO:0033120] (biological process) Subtypes: positive regulation of mRNA splicing, via spliceosome [GO:0048026] Relationships: is a type of positive regulation of gene expression [GO:0010628]; is a type of GO:0043484; positively regulates GO:0008380 Definition: Any process that activates or increases the frequency, rate or extent of RNA splicing. Sources: GOC:mah